{
  "gene_symbol": "SESTD1",
  "gene": "UniProtKB:Q86VW0",
  "term_id": "GO:0043325",
  "term_label": "phosphatidylinositol-3,4-bisphosphate binding",
  "gene_name": "SEC14 domain and spectrin repeat-containing protein 1"
}